{
  "gene": "UniProtKB:Q9NP77",
  "gene_name": "RNA polymerase II subunit A C-terminal domain phosphatase SSU72",
  "gene_symbol": "SSU72",
  "term_id": "GO:0005847",
  "term_label": "mRNA cleavage and polyadenylation specificity factor complex"
}